{
  "term_label": "axon",
  "gene_symbol": "RUFY3",
  "gene_name": "Protein RUFY3",
  "term_id": "GO:0030424",
  "gene": "UniProtKB:Q7L099"
}